iron import into cell [GO:0033212] (biological process) Also known as: ferrous ion import, ferrous iron import, ferrous iron uptake, iron assimilation Subtypes: reductive iron assimilation [GO:0033215], iron ion import across plasma membrane [GO:0098711], endocytic iron import into cell [GO:0140298], heme import into cell [GO:0140420], GO:0180060 Definition: The directed movement of iron ions from outside of a cell into the cytoplasmic compartment. This may occur via transport across the plasma membrane or via endocytosis. References: PMID:18622392, PMID:23192658 Sources: Wikipedia:Human_iron_metabolism Relationships: is a type of iron ion transport [GO:0006826]; is a type of intracellular iron ion homeostasis [GO:0006879]; is a type of establishment of localization in cell [GO:0051649]